{
  "gene": "UniProtKB:Q9HAY6",
  "term_id": "GO:0042574",
  "term_label": "retinal metabolic process",
  "gene_name": "Beta,beta-carotene 15,15'-dioxygenase",
  "gene_symbol": "BCO1"
}